{
  "gene": "UniProtKB:Q5T5A4",
  "gene_name": "Cilia- and flagella-associated protein 276",
  "term_label": "Unknown molecular function",
  "gene_symbol": "CFAP276",
  "term_id": "UNKNOWN:0001"
}